{
  "gene": "UniProtKB:P61978",
  "gene_symbol": "HNRNPK",
  "gene_name": "Heterogeneous nuclear ribonucleoprotein K",
  "term_label": "mRNA binding",
  "term_id": "GO:0003729"
}